{
  "gene_symbol": "DECR1",
  "term_label": "fatty acid beta-oxidation",
  "gene": "UniProtKB:Q16698",
  "term_id": "GO:0006635",
  "gene_name": "2,4-dienoyl-CoA reductase [(3E)-enoyl-CoA-producing], mitochondrial"
}